{
  "gene": "UniProtKB:Q13634",
  "gene_name": "Cadherin-18",
  "term_label": "adherens junction",
  "gene_symbol": "CDH18",
  "term_id": "GO:0005912"
}